{
  "gene_name": "Ciliogenesis and planar polarity effector 1",
  "gene": "UniProtKB:Q9H799",
  "term_id": "GO:0060271",
  "gene_symbol": "CPLANE1",
  "term_label": "cilium assembly"
}